{
  "term_label": "mitochondrion",
  "gene_symbol": "YARS2",
  "term_id": "GO:0005739",
  "gene": "UniProtKB:Q9Y2Z4",
  "gene_name": "Tyrosine--tRNA ligase, mitochondrial"
}